{
  "gene_name": "Synaptophysin-like protein 1",
  "term_id": "GO:0030672",
  "gene_symbol": "SYPL1",
  "gene": "UniProtKB:Q16563",
  "term_label": "synaptic vesicle membrane"
}